{
  "term_label": "nucleus",
  "gene_symbol": "FAM53B",
  "gene": "UniProtKB:Q14153",
  "term_id": "GO:0005634",
  "gene_name": "Protein FAM53B"
}